positive regulation of protein refolding [GO:1904592] (biological process) Definition: Any process that activates or increases the frequency, rate or extent of protein refolding. References: PMID:11360998 Sources: GOC:TermGenie, GO_REF:0000058 Also known as: up regulation of protein refolding, up-regulation of protein refolding, upregulation of protein refolding, activation of protein refolding, activation of heat shock protein activity, positive regulation of heat shock protein activity, up regulation of heat shock protein activity, up-regulation of heat shock protein activity, upregulation of heat shock protein activity Relationships: is a type of regulation of protein refolding [GO:0061083]; is a type of positive regulation of protein folding [GO:1903334]; positively regulates GO:0042026